{
  "term_label": "cytosol",
  "gene_name": "Dedicator of cytokinesis protein 6",
  "gene_symbol": "DOCK6",
  "gene": "UniProtKB:Q96HP0",
  "term_id": "GO:0005829"
}